{
  "gene_name": "Anoctamin-3",
  "term_label": "phospholipid scramblase activity",
  "gene_symbol": "ANO3",
  "term_id": "GO:0017128",
  "gene": "UniProtKB:Q9BYT9"
}